positive regulation of octadecene biosynthetic process [GO:1900916] (biological process) Relationships: is_a positive regulation of olefin biosynthetic process [GO:1900913]; is a type of regulation of octadecene biosynthetic process [GO:1900914]; RO_0002213 octadecene biosynthetic process [GO:1900682] Sources: GOC:TermGenie, GOC:mengo_curators Also known as: up regulation of octadecene biosynthetic process, up-regulation of octadecene biosynthetic process, upregulation of octadecene biosynthetic process, activation of octadecene biosynthetic process, activation of 1-octadecene biosynthetic process, activation of octadecene anabolism, activation of octadecene biosynthesis, activation of octadecene formation, activation of octadecene synthesis, positive regulation of 1-octadecene biosynthetic process, positive regulation of octadecene anabolism, positive regulation of octadecene biosynthesis, positive regulation of octadecene formation, positive regulation of octadecene synthesis, up regulation of 1-octadecene biosynthetic process, up regulation of octadecene anabolism, up regulation of octadecene biosynthesis, up regulation of octadecene formation, up regulation of octadecene synthesis, up-regulation of 1-octadecene biosynthetic process, up-regulation of octadecene anabolism, up-regulation of octadecene biosynthesis, up-regulation of octadecene formation, up-regulation of octadecene synthesis, upregulation of 1-octadecene biosynthetic process, upregulation of octadecene anabolism, upregulation of octadecene biosynthesis, upregulation of octadecene formation, upregulation of octadecene synthesis Definition: Any process that activates or increases the frequency, rate or extent of octadecene biosynthetic process.